{
  "term_id": "GO:0000122",
  "gene": "UniProtKB:O15479",
  "gene_name": "Melanoma-associated antigen B2",
  "gene_symbol": "MAGEB2",
  "term_label": "negative regulation of transcription by RNA polymerase II"
}